{
  "gene": "UniProtKB:Q9HCC8",
  "gene_name": "Glycerophosphoinositol inositolphosphodiesterase GDPD2",
  "term_label": "Unknown biological process",
  "term_id": "UNKNOWN:0002",
  "gene_symbol": "GDPD2"
}